meiotic gene conversion [GO:0006311] (BP) Sources: ISBN:0815316194 Definition: The cell cycle process in which genetic information is transferred from one helix to another. It often occurs in association with general genetic recombination events, and is believed to be a straightforward consequence of the mechanisms of general recombination and DNA repair. For example, meiosis might yield three copies of the maternal version of an allele and only one copy of the paternal allele, indicating that one of the two copies of the paternal allele has been changed to a copy of the maternal allele. Relationships: is a type of gene conversion [GO:0035822]; is a type of meiosis I cell cycle process [GO:0061982] Also known as: gene conversion without reciprocal crossover